{
  "gene_name": "Probable ATP-dependent RNA helicase DDX46",
  "term_label": "mRNA splicing, via spliceosome",
  "term_id": "GO:0000398",
  "gene_symbol": "DDX46",
  "gene": "UniProtKB:Q7L014"
}